{
  "term_label": "citrate transmembrane transporter activity",
  "gene_symbol": "SLC13A5",
  "gene": "UniProtKB:Q86YT5",
  "term_id": "GO:0015137",
  "gene_name": "Na(+)_citrate cotransporter"
}